{
  "gene": "UniProtKB:O60341",
  "term_id": "GO:0003682",
  "term_label": "chromatin binding",
  "gene_symbol": "KDM1A",
  "gene_name": "Lysine-specific histone demethylase 1A"
}